{
  "term_id": "GO:0007507",
  "gene_symbol": "CCM2",
  "gene": "UniProtKB:Q9BSQ5",
  "term_label": "heart development",
  "gene_name": "Cerebral cavernous malformations 2 protein"
}